{
  "gene_symbol": "DYNC2I1",
  "term_id": "GO:0045503",
  "gene_name": "Cytoplasmic dynein 2 intermediate chain 1",
  "term_label": "dynein light chain binding",
  "gene": "UniProtKB:Q8WVS4"
}